{
  "gene": "UniProtKB:Q6DKI2",
  "term_label": "galactoside binding",
  "gene_symbol": "LGALS9C",
  "gene_name": "Galectin-9C",
  "term_id": "GO:0016936"
}